long-chain fatty acid transporting porin activity [GO:0015483] (molecular function) Definition: Enables the transfer of a long-chain fatty acid from one side of a membrane to the other. A long-chain fatty acid has an aliphatic tail containing 13 to 22 carbons. This transporter is a porin and so enables the energy independent passage of substances, sized less than 1000 Da, across a membrane. The transmembrane portions of porins consist exclusively of beta-strands which form a beta-barrel. They are found in the outer membranes of Gram-negative bacteria, mitochondria, plastids and possibly acid-fast Gram-positive bacteria. Sources: GOC:mtg_transport, TC:1.B.9.1.1 Note: While there is not universal consensus on the lengths of short-, medium-, long- and very-long-chain fatty acids, the GO uses the definitions in ChEBI (see CHEBI:26666, CHEBI:59554, CHEBI:15904 and CHEBI:27283). Relationships: is a type of long-chain fatty acid transmembrane transporter activity [GO:0005324]; is a type of porin activity [GO:0015288]